{
  "gene_symbol": "ZNF574",
  "term_id": "GO:0006357",
  "gene_name": "Zinc finger protein 574",
  "gene": "UniProtKB:Q6ZN55",
  "term_label": "regulation of transcription by RNA polymerase II"
}